opheline kinase activity [GO:0050154] (molecular function) Definition: Catalysis of the reaction: ATP + guanidinoethyl methyl phosphate = N'-phosphoguanidinoethyl methylphosphate + ADP + 2 H+. Sources: EC:2.7.3.7, RHEA:17553 Also known as: ATP:guanidinoethyl-methyl-phosphate phosphotransferase activity Relationships: is a type of kinase activity [GO:0016301]; is a type of GO:0016775